cholecystokinin signaling pathway [GO:0038188] (biological process) Relationships: is_a GO:0007186 References: PMID:11181948 Sources: GOC:jc Subtypes: positive regulation of pancreatic amylase secretion by cholecystokinin signaling pathway [GO:1902279] Definition: A G protein-coupled receptor signaling pathway initiated by cholecystokinin binding to its receptor on the surface of a target cell, and ending with the regulation of a downstream cellular process, e.g. transcription. Also known as: CCK signaling, cholecystokinin receptor signaling pathway